{
  "term_label": "Unknown cellular component",
  "term_id": "UNKNOWN:0003",
  "gene": "UniProtKB:Q9NRQ5",
  "gene_name": "Single-pass membrane and coiled-coil domain-containing protein 4",
  "gene_symbol": "SMCO4"
}